{
  "gene": "UniProtKB:P20853",
  "term_id": "GO:0016712",
  "gene_symbol": "CYP2A7",
  "term_label": "oxidoreductase activity, acting on paired donors, with incorporation or reduction of molecular oxygen, reduced flavin or flavoprotein as one donor, and incorporation of one atom of oxygen",
  "gene_name": "Cytochrome P450 2A7"
}